negative regulation of receptor signaling pathway via JAK-STAT [GO:0046426] (BP) Subtypes: negative regulation of tyrosine phosphorylation of STAT protein [GO:0042532] Also known as: down regulation of JAK-STAT cascade, down-regulation of JAK-STAT cascade, downregulation of JAK-STAT cascade, inhibition of JAK-STAT cascade, negative regulation of STAT protein import into nucleus, negative regulation of STAT protein nuclear translocation Relationships: is a type of regulation of receptor signaling pathway via JAK-STAT [GO:0046425]; is a type of negative regulation of receptor signaling pathway via STAT [GO:1904893]; negatively regulates cell surface receptor signaling pathway via JAK-STAT [GO:0007259] Sources: GOC:bf Definition: Any process that stops, prevents, or reduces the frequency, rate or extent of a receptor signaling pathway via JAK-STAT.